{
  "gene_name": "Serine_threonine-protein phosphatase 2A 55 kDa regulatory subunit B alpha isoform",
  "term_label": "cytosol",
  "gene": "UniProtKB:P63151",
  "gene_symbol": "PPP2R2A",
  "term_id": "GO:0005829"
}